{
  "gene_name": "Transcription factor SOX-1",
  "term_id": "GO:0000122",
  "gene_symbol": "SOX1",
  "term_label": "negative regulation of transcription by RNA polymerase II",
  "gene": "UniProtKB:O00570"
}